basal plasma membrane [GO:0009925] (cellular component) Sources: GOC:go_curators Definition: The region of the plasma membrane located at the basal end of the cell. Often used in reference to animal polarized epithelial membranes, where the basal membrane is the part attached to the extracellular matrix, or in plant cells, where the basal membrane is defined with respect to the zygotic axis. Relationships: is a type of plasma membrane region [GO:0098590]; is part of basal part of cell [GO:0045178]